{
  "term_id": "GO:0032580",
  "gene": "UniProtKB:Q0D2H9",
  "term_label": "Golgi cisterna membrane",
  "gene_symbol": "GOLGA8DP",
  "gene_name": "Putative golgin subfamily A member 8D"
}